{
  "gene_name": "Alpha-catulin",
  "term_id": "UNKNOWN:0001",
  "term_label": "Unknown molecular function",
  "gene": "UniProtKB:Q9UBT7",
  "gene_symbol": "CTNNAL1"
}